neurotransmitter receptor activity involved in regulation of postsynaptic cytosolic calcium ion concentration [GO:0099583] (molecular function) Relationships: is a type of postsynaptic neurotransmitter receptor activity [GO:0098960]; is part of regulation of postsynaptic cytosolic calcium ion concentration [GO:0099566] Definition: Any neurotransmitter receptor activity that is involved in regulating the concentration of calcium in the postsynaptic cytosol. Subtypes: GO:0098872 Also known as: neurotransmitter receptor activity involved in regulation of postsynaptic cytosolic calcium levels Sources: GOC:dos